{
  "gene_name": "Cell cycle checkpoint control protein RAD9B",
  "term_id": "GO:0006281",
  "gene_symbol": "RAD9B",
  "term_label": "DNA repair",
  "gene": "UniProtKB:Q6WBX8"
}